{
  "gene_name": "Putative solute carrier family 26 member 10P",
  "term_label": "chloride transmembrane transporter activity",
  "gene_symbol": "SLC26A10P",
  "term_id": "GO:0015108",
  "gene": "UniProtKB:Q8NG04"
}